{
  "gene_name": "Poly(A)-specific ribonuclease PARN",
  "gene_symbol": "PARN",
  "term_id": "GO:1990432",
  "term_label": "siRNA 3'-end processing",
  "gene": "UniProtKB:O95453"
}